ferredoxin-NADP+ reductase activity [GO:0004324] (molecular function) Also known as: ferredoxin-NADP reductase activity, NADP:ferredoxin oxidoreductase activity, NADPH:ferredoxin oxidoreductase activity, TPNH-ferredoxin reductase activity, ferredoxin-NADP oxidoreductase activity, ferredoxin-NADP-oxidoreductase activity, ferredoxin-TPN reductase activity, ferredoxin-nicotinamide adenine dinucleotide phosphate reductase activity, ferredoxin-nicotinamide-adenine dinucleotide phosphate (oxidized) reductase activity, ferredoxin:NADP+ oxidoreductase activity, reduced nicotinamide adenine dinucleotide phosphate-adrenodoxin reductase activity Definition: Catalysis of the reaction: 2 reduced [2Fe-2S]-[ferredoxin] + NADP+ + H+ = 2 oxidized [2Fe-2S]-[ferredoxin] + NADPH. Sources: RHEA:20125 Relationships: is a type of ferredoxin-[NAD(P)H] reductase activity [GO:0008937]